{
  "gene_name": "Melatonin receptor type 1A",
  "gene_symbol": "MTNR1A",
  "gene": "UniProtKB:P48039",
  "term_id": "GO:0007193",
  "term_label": "adenylate cyclase-inhibiting G protein-coupled receptor signaling pathway"
}